phosphatidylinositol 3-kinase regulatory subunit binding [GO:0036312] (molecular function) References: PMID:20505341 Sources: GOC:bf Relationships: is a type of phosphatidylinositol 3-kinase binding [GO:0043548] Also known as: PI3K regulatory subunit binding, p85 binding Definition: Binding to a regulatory subunit of phosphatidylinositol 3-kinase. The regulatory subunit associates with the catalytic subunit to regulate both its activity and subcellular location.